{
  "term_id": "GO:0001889",
  "gene_symbol": "PRKCSH",
  "term_label": "liver development",
  "gene": "UniProtKB:P14314",
  "gene_name": "Glucosidase 2 subunit beta"
}